perivitelline space [GO:0098595] (cellular component) Sources: GOC:dos Relationships: is a type of extracellular region [GO:0005576] Definition: The space between the membrane of an oocyte and a surrounding membranous structure (zona pellucida or perivitelline membrane).